germ-line processes downstream of sex determination signal [GO:0007547] (biological process) Sources: GOC:ems Definition: The events determining the germ-line sexual phenotype after the initial transmission of that phenotype to germ-line-specific information pathways. Relationships: is a type of processes downstream of sex determination signal [GO:0007545]; is part of germ-line sex determination [GO:0018992]